{
  "term_label": "regulation of innate immune response",
  "gene": "UniProtKB:Q496F6",
  "gene_symbol": "CD300E",
  "gene_name": "CMRF35-like molecule 2",
  "term_id": "GO:0045088"
}